negative regulation of tyrosine phosphorylation of STAT protein [GO:0042532] (biological process) Also known as: down regulation of tyrosine phosphorylation of STAT protein, down-regulation of tyrosine phosphorylation of STAT protein, downregulation of tyrosine phosphorylation of STAT protein, down regulation of tyrosine phosphorylation of Stat1 protein, down regulation of tyrosine phosphorylation of Stat2 protein, down regulation of tyrosine phosphorylation of Stat3 protein, down regulation of tyrosine phosphorylation of Stat4 protein, down regulation of tyrosine phosphorylation of Stat5 protein, down regulation of tyrosine phosphorylation of Stat6 protein, down regulation of tyrosine phosphorylation of Stat7 protein, down-regulation of tyrosine phosphorylation of Stat1 protein, down-regulation of tyrosine phosphorylation of Stat2 protein, down-regulation of tyrosine phosphorylation of Stat3 protein, down-regulation of tyrosine phosphorylation of Stat4 protein, down-regulation of tyrosine phosphorylation of Stat5 protein, down-regulation of tyrosine phosphorylation of Stat6 protein, down-regulation of tyrosine phosphorylation of Stat7 protein, downregulation of tyrosine phosphorylation of Stat1 protein, downregulation of tyrosine phosphorylation of Stat2 protein, downregulation of tyrosine phosphorylation of Stat3 protein, downregulation of tyrosine phosphorylation of Stat4 protein, downregulation of tyrosine phosphorylation of Stat5 protein, downregulation of tyrosine phosphorylation of Stat6 protein, downregulation of tyrosine phosphorylation of Stat7 protein, inhibition of tyrosine phosphorylation of STAT protein, inhibition of tyrosine phosphorylation of Stat1 protein, inhibition of tyrosine phosphorylation of Stat2 protein, inhibition of tyrosine phosphorylation of Stat3 protein, inhibition of tyrosine phosphorylation of Stat4 protein, inhibition of tyrosine phosphorylation of Stat5 protein, inhibition of tyrosine phosphorylation of Stat6 protein, inhibition of tyrosine phosphorylation of Stat7 protein, negative regulation of tyrosine phosphorylation of Stat1 protein, negative regulation of tyrosine phosphorylation of Stat2 protein, negative regulation of tyrosine phosphorylation of Stat3 protein, negative regulation of tyrosine phosphorylation of Stat4 protein, negative regulation of tyrosine phosphorylation of Stat5 protein, negative regulation of tyrosine phosphorylation of Stat6 protein, negative regulation of tyrosine phosphorylation of Stat7 protein Definition: Any process that stops, prevents, or reduces the frequency, rate or extent of the introduction of a phosphate group to a tyrosine residue of a STAT (Signal Transducer and Activator of Transcription) protein. Relationships: is a type of regulation of tyrosine phosphorylation of STAT protein [GO:0042509]; is a type of negative regulation of receptor signaling pathway via JAK-STAT [GO:0046426]; is a type of negative regulation of peptidyl-tyrosine phosphorylation [GO:0050732]; negatively regulates tyrosine phosphorylation of STAT protein [GO:0007260] References: PMID:11426647 Sources: GOC:jl